distal tubule development [GO:0072017] (biological process) Definition: The process whose specific outcome is the progression of the distal tubule over time, from its formation to the mature structure. In mammals, the distal tubule is a nephron tubule that begins at the macula densa and extends to the connecting tubule. Sources: GOC:mtg_kidney_jan10 Subtypes: pronephric distal tubule development [GO:0035777], GO:0061274, metanephric distal tubule development [GO:0072235] Relationships: is a type of GO:0072080